{
  "term_label": "membrane",
  "gene_name": "Protein mono-ADP-ribosyltransferase PARP6",
  "term_id": "GO:0016020",
  "gene_symbol": "PARP6",
  "gene": "UniProtKB:Q2NL67"
}